{
  "gene_name": "G2_mitotic-specific cyclin-B2",
  "gene": "UniProtKB:O95067",
  "term_id": "GO:0000082",
  "gene_symbol": "CCNB2",
  "term_label": "G1/S transition of mitotic cell cycle"
}